{
  "term_label": "Unknown molecular function",
  "gene": "UniProtKB:A6NGB9",
  "gene_name": "WAS_WASL-interacting protein family member 3",
  "gene_symbol": "WIPF3",
  "term_id": "UNKNOWN:0001"
}